{
  "gene_symbol": "THAP4",
  "term_id": "UNKNOWN:0001",
  "term_label": "Unknown molecular function",
  "gene": "UniProtKB:Q8WY91",
  "gene_name": "Peroxynitrite isomerase THAP4"
}